cellular response to curcumin [GO:1904644] (biological process) References: PMID:24755072 Sources: GOC:TermGenie, GO_REF:0000071 Definition: Any process that results in a change in state or activity of a cell (in terms of movement, secretion, enzyme production, gene expression, etc.) as a result of a curcumin stimulus. Relationships: is a type of GO:0071362; is a type of cellular response to ketone [GO:1901655]; is a type of GO:1904643